interneuron axon guidance [GO:0097376] (biological process) Sources: CL:0000099, GOC:pr Subtypes: spinal cord interneuron axon guidance [GO:0097377] Definition: The process in which the migration of an axon growth cone of an interneuron is directed to a specific target site in response to a combination of attractive and repulsive cues. An interneuron is any neuron which is not motor or sensory. Interneurons may also refer to neurons whose axons remain within a particular brain region, as contrasted with projection neurons which have axons projecting to other brain regions. Relationships: is a type of axon guidance [GO:0007411]